{
  "term_id": "GO:0006357",
  "term_label": "regulation of transcription by RNA polymerase II",
  "gene_name": "Zinc finger protein Pegasus",
  "gene_symbol": "IKZF5",
  "gene": "UniProtKB:Q9H5V7"
}